{
  "gene_symbol": "GNA11",
  "gene": "UniProtKB:P29992",
  "term_id": "GO:0007188",
  "gene_name": "Guanine nucleotide-binding protein subunit alpha-11",
  "term_label": "adenylate cyclase-modulating G protein-coupled receptor signaling pathway"
}